{
  "gene_name": "Ubiquitin carboxyl-terminal hydrolase 47",
  "term_label": "cysteine-type deubiquitinase activity",
  "gene_symbol": "USP47",
  "term_id": "GO:0004843",
  "gene": "UniProtKB:Q96K76"
}